{
  "gene": "UniProtKB:A0FGR9",
  "term_label": "endoplasmic reticulum membrane",
  "gene_name": "Extended synaptotagmin-3",
  "term_id": "GO:0005789",
  "gene_symbol": "ESYT3"
}